{
  "gene": "UniProtKB:Q9UL18",
  "term_id": "GO:0035194",
  "gene_name": "Protein argonaute-1",
  "gene_symbol": "AGO1",
  "term_label": "regulatory ncRNA-mediated post-transcriptional gene silencing"
}